{
  "gene": "UniProtKB:Q7Z4L0",
  "gene_name": "Cytochrome c oxidase subunit 8C, mitochondrial",
  "gene_symbol": "COX8C",
  "term_id": "GO:0045277",
  "term_label": "respiratory chain complex IV"
}